{
  "term_id": "GO:0005576",
  "gene_name": "Follistatin-related protein 4",
  "gene": "UniProtKB:Q6MZW2",
  "term_label": "extracellular region",
  "gene_symbol": "FSTL4"
}